viral terminase, small subunit [GO:0097710] (cellular component) Also known as: virus terminase, small subunit Note: This term should only be used when the small subunit consists of more than one polypeptide. Relationships: is a type of protein-containing complex [GO:0032991]; is part of viral terminase complex [GO:0043493] Definition: The part of the viral terminase complex that acts as a phage DNA-recognition component and regulates the activity of the large subunit. The small subunit usually assembles as a heterooligomer with the large subunit. References: PMID:18687036 Sources: GOC:ch, GOC:jh2